{
  "gene_name": "Potassium voltage-gated channel subfamily H member 1",
  "gene": "UniProtKB:O95259",
  "term_label": "voltage-gated potassium channel complex",
  "term_id": "GO:0008076",
  "gene_symbol": "KCNH1"
}